{
  "gene_name": "Fibroblast growth factor 4",
  "term_label": "extracellular space",
  "term_id": "GO:0005615",
  "gene_symbol": "FGF4",
  "gene": "UniProtKB:P08620"
}